{
  "term_label": "dense core granule",
  "gene": "UniProtKB:Q86SS6",
  "gene_symbol": "SYT9",
  "term_id": "GO:0031045",
  "gene_name": "Synaptotagmin-9"
}